{
  "gene_symbol": "CREB3L2",
  "gene_name": "Cyclic AMP-responsive element-binding protein 3-like protein 2",
  "term_label": "DNA-binding transcription factor activity, RNA polymerase II-specific",
  "term_id": "GO:0000981",
  "gene": "UniProtKB:Q70SY1"
}